{
  "gene_name": "Histone-lysine N-methyltransferase SUV39H1",
  "gene_symbol": "SUV39H1",
  "term_label": "histone H3K9 methyltransferase activity",
  "gene": "UniProtKB:O43463",
  "term_id": "GO:0046974"
}